transcription elongation by RNA polymerase II [GO:0006368] (biological process) Definition: The extension of an RNA molecule after transcription pausing and promoter clearance at an RNA polymerase II promoter by the addition of ribonucleotides catalyzed by RNA polymerase II. Regulation: positively regulated by GO:0032968; regulated by regulation of transcription elongation by RNA polymerase II [GO:0034243]; RO_0002212 by GO:0034244 Sources: GOC:mah, GOC:txnOH Relationships: is a type of GO:0006354; is part of GO:0006366 Also known as: RNA elongation from Pol II promoter, transcription elongation by RNA polymerase II promoter, transcription elongation from RNA polymerase II promoter, RNA polymerase II transcription elongation factor activity